regulation of sodium ion transport [GO:0002028] (biological process) Relationships: is_a regulation of metal ion transport [GO:0010959]; regulates sodium ion transport [GO:0006814] Also known as: regulation of Na+ transport, regulation of sodium transport Sources: GOC:dph Subtypes: GO:0010765, GO:0010766, regulation of sodium ion transmembrane transport [GO:1902305] Definition: Any process that modulates the frequency, rate or extent of the directed movement of sodium ions (Na+) into, out of or within a cell, or between cells, by means of some agent such as a transporter or pore.